{
  "term_label": "heart morphogenesis",
  "gene_name": "Nipped-B-like protein",
  "gene_symbol": "NIPBL",
  "gene": "UniProtKB:Q6KC79",
  "term_id": "GO:0003007"
}